{
  "term_label": "endoplasmic reticulum",
  "gene_symbol": "SPTLC1",
  "gene": "UniProtKB:O15269",
  "gene_name": "Serine palmitoyltransferase 1",
  "term_id": "GO:0005783"
}